{
  "term_label": "Unknown cellular component",
  "gene_name": "Protein SCO1 homolog, mitochondrial",
  "gene": "UniProtKB:O75880",
  "gene_symbol": "SCO1",
  "term_id": "UNKNOWN:0003"
}